{
  "gene_name": "Putative solute carrier family 26 member 10P",
  "gene_symbol": "SLC26A10P",
  "term_id": "GO:0019531",
  "term_label": "oxalate transmembrane transporter activity",
  "gene": "UniProtKB:Q8NG04"
}